regulation of intracellular steroid hormone receptor signaling pathway [GO:0033143] (biological process) Sources: GOC:mah Subtypes: negative regulation of intracellular steroid hormone receptor signaling pathway [GO:0033144], positive regulation of intracellular steroid hormone receptor signaling pathway [GO:0033145], regulation of intracellular estrogen receptor signaling pathway [GO:0033146], regulation of androgen receptor signaling pathway [GO:0060765], regulation of ecdysone receptor signaling pathway [GO:0120141], GO:2000322 Also known as: regulation of steroid hormone receptor signaling pathway, regulation of steroid hormone receptor signalling pathway Relationships: is a type of regulation of intracellular signal transduction [GO:1902531]; RO_0002211 nuclear receptor-mediated steroid hormone signaling pathway [GO:0030518] Definition: Any process that modulates the frequency, rate or extent of the activity of any intracellular steroid hormone receptor signaling pathway.